phosphoric ester hydrolase activity [GO:0042578] (molecular function) Subtypes: phosphoric diester hydrolase activity [GO:0008081], phosphatase activity [GO:0016791], triphosphoric monoester hydrolase activity [GO:0016793], GO:0016794, phosphoric triester hydrolase activity [GO:0016795] Relationships: is a type of GO:0016788 Definition: Catalysis of the reaction: RPO-R' + H2O = RPOOH + R'H. This reaction is the hydrolysis of any phosphoric ester bond, any ester formed from orthophosphoric acid, O=P(OH)3. Sources: GOC:jl